beige fat cell differentiation [GO:0160274] (biological process) Definition: The process in which a white fat cell acquires specialized features of a beige adipocyte. Beige adipocytes reside within white adipose tissue and can be induced to produce heat in response to cold exposure or certain stimuli, resembling brown adipocytes. Relationships: is a type of GO:0045444 References: PMID:24439384 Regulation: negatively regulated by GO:0160276 Also known as: brite fat cell differentiation, brown-in white fat cell differentiation